CoA-synthesizing protein complex [GO:1990143] (cellular component) Definition: A multisubunit complex likely involved in the synthesis of coenzyme A (CoA). In S. cerevisiae, the complex consists of at least Cab2, Cab3, Cab4 and Cab5 but may also include Sis2 and Vhs3. The latter subunits are shared by the GO:0071513 phosphopantothenoylcysteine decarboxylase complex that catalyses the third step of the coenzyme A (CoA) biosynthetic pathway. References: PMID:23789928 Sources: GOC:rb Also known as: CoA-SPC, coenzyme A-synthesizing protein complex Relationships: is a type of catalytic complex [GO:1902494]